positive regulation of adenylate cyclase-activating adrenergic receptor signaling pathway [GO:0071879] (biological process) Also known as: positive regulation of adrenergic receptor signaling pathway, positive regulation of adrenergic receptor signalling pathway Sources: GOC:BHF, GOC:mah Definition: Any process that activates or increases the frequency, rate or extent of the adenylate cyclase-activating adrenergic receptor protein signaling pathway. An adrenergic receptor signaling pathway is the series of molecular signals generated as a consequence of an adrenergic receptor binding to one of its physiological ligands. Relationships: is a type of GO:0045745; positively regulates adrenergic receptor signaling pathway [GO:0071875] Subtypes: GO:0140196